L-erythro-3-methylmalyl-CoA dehydratase activity [GO:0043960] (molecular function) Definition: Catalysis of the reaction: L-erythro-3-methylmalyl-CoA = mesaconyl-CoA + H2O. Relationships: is a type of hydro-lyase activity [GO:0016836] Sources: GOC:jl